fatty acid beta-oxidation [GO:0006635] (BP) Sources: GOC:mah, ISBN:0198506732 Regulation: regulated by GO:0031998; negatively regulated by GO:0031999; positively regulated by GO:0032000 Definition: A fatty acid oxidation process that results in the complete oxidation of a long-chain fatty acid. Fatty acid beta-oxidation begins with the addition of coenzyme A to a fatty acid, and occurs by successive cycles of reactions during each of which the fatty acid is shortened by a two-carbon fragment removed as acetyl coenzyme A; the cycle continues until only two or three carbons remain (as acetyl-CoA or propionyl-CoA respectively). Subtypes: fatty acid beta-oxidation using acyl-CoA dehydrogenase [GO:0033539], fatty acid beta-oxidation using acyl-CoA oxidase [GO:0033540], fatty acid beta-oxidation, unsaturated, odd number [GO:0033541], fatty acid beta-oxidation, unsaturated, even number [GO:0033542] Relationships: is_a GO:0009062; is a type of GO:0019395; has part fatty acid ligase activity [GO:0015645]